regulation of response to formic acid [GO:1901460] (biological process) Definition: Any process that modulates the frequency, rate or extent of response to formic acid. Relationships: is a type of GO:0048583; regulates response to formic acid [GO:1901425] Sources: GOC:TermGenie, GOC:mengo_curators Subtypes: negative regulation of response to formic acid [GO:1901461], positive regulation of response to formic acid [GO:1901462]